{
  "gene_name": "Transmembrane anterior posterior transformation protein 1 homolog",
  "term_label": "endoplasmic reticulum membrane",
  "gene": "UniProtKB:Q6NXT6",
  "term_id": "GO:0005789",
  "gene_symbol": "TAPT1"
}